{
  "gene_symbol": "SORT1",
  "term_id": "GO:0030379",
  "gene_name": "Sortilin",
  "term_label": "neurotensin receptor activity, non-G protein-coupled",
  "gene": "UniProtKB:Q99523"
}